branched-chain amino acid:sodium symporter activity [GO:0015657] (MF) Definition: Enables the transfer of a solute or solutes from one side of a membrane to the other according to the reaction: branched-chain amino acid(out) + cation(out) = branched-chain amino acid(in) + cation(in). Relationships: is a type of organic acid:sodium symporter activity [GO:0005343]; is a type of branched-chain amino acid transmembrane transporter activity [GO:0015658] Sources: TC:2.A.26.1.1